{
  "gene_name": "Protein argonaute-4",
  "term_id": "GO:0016442",
  "gene": "UniProtKB:Q9HCK5",
  "term_label": "RISC complex",
  "gene_symbol": "AGO4"
}